{
  "term_id": "GO:0005178",
  "gene": "UniProtKB:P32942",
  "gene_name": "Intercellular adhesion molecule 3",
  "gene_symbol": "ICAM3",
  "term_label": "integrin binding"
}